{
  "term_id": "GO:0051604",
  "gene_symbol": "PRPH2",
  "gene": "UniProtKB:P23942",
  "gene_name": "Peripherin-2",
  "term_label": "protein maturation"
}